{
  "gene_symbol": "CDCA7L",
  "gene_name": "Cell division cycle-associated 7-like protein",
  "term_label": "Unknown biological process",
  "term_id": "UNKNOWN:0002",
  "gene": "UniProtKB:Q96GN5"
}